regulation of antigen receptor-mediated signaling pathway [GO:0050854] (biological process) Sources: GOC:ai Subtypes: regulation of B cell receptor signaling pathway [GO:0050855], regulation of T cell receptor signaling pathway [GO:0050856], positive regulation of antigen receptor-mediated signaling pathway [GO:0050857], negative regulation of antigen receptor-mediated signaling pathway [GO:0050858] Also known as: regulation of antigen receptor mediated signalling pathway Relationships: is a type of regulation of signal transduction [GO:0009966]; is a type of regulation of immune response [GO:0050776]; regulates GO:0050851 Definition: Any process that modulates the frequency, rate or extent of signaling pathways initiated by the cross-linking of an antigen receptor on a B- or T cell.